megasporocyte nucleus [GO:0043076] (cellular component) Sources: GOC:jl, ISBN:0618254153 Subtypes: polar nucleus [GO:0043078], antipodal cell nucleus [GO:0043079], megagametophyte egg cell nucleus [GO:0043082] Relationships: is a type of nucleus [GO:0005634] Also known as: megaspore mother cell nucleus Definition: The nucleus of a megasporocyte, a diploid cell that undergoes meiosis to produce four megaspores, and its descendents.